B cell antigen processing and presentation following pinocytosis [GO:0002421] (biological process) Definition: B cell antigen processing and presentation which is initiated by uptake of antigen via pinocytosis. References: PMID:7543530 Sources: GOC:add Also known as: B lymphocyte antigen processing and presentation following pinocytosis, B-cell antigen processing and presentation following pinocytosis, B-lymphocyte antigen processing and presentation following pinocytosis Relationships: is a type of GO:0002450; is_a antigen processing and presentation following pinocytosis [GO:0002746]